{
  "term_id": "GO:0007616",
  "gene_symbol": "LRRN4",
  "gene_name": "Leucine-rich repeat neuronal protein 4",
  "gene": "UniProtKB:Q8WUT4",
  "term_label": "long-term memory"
}